{
  "gene": "UniProtKB:P55327",
  "gene_symbol": "TPD52",
  "gene_name": "Tumor protein D52",
  "term_label": "Unknown molecular function",
  "term_id": "UNKNOWN:0001"
}